MutLgamma complex [GO:0097587] (cellular component) Definition: A heterodimer involved in the recognition of base-base and small insertion/deletion mismatches. In S. cerevisiae the complex consists of two subunits, Mlh1 and Mlh3. References: PMID:10570173 Sources: GOC:jd Relationships: is a type of mismatch repair complex [GO:0032300]